negative regulation of protein maturation [GO:1903318] (biological process) Definition: Any process that stops, prevents or reduces the frequency, rate or extent of protein maturation. Subtypes: GO:0010955, negative regulation of N-terminal peptidyl-methionine acetylation [GO:1904664], negative regulation of protein activation cascade [GO:2000258], GO:2000760 Also known as: down regulation of protein maturation, down-regulation of protein maturation, downregulation of protein maturation, inhibition of protein maturation Relationships: is_a GO:0010629; is a type of negative regulation of protein metabolic process [GO:0051248]; is a type of GO:1903317; negatively regulates protein maturation [GO:0051604] Sources: GOC:TermGenie, GOC:vw, GO_REF:0000058